{
  "gene_name": "NK1 transcription factor-related protein 1",
  "gene": "UniProtKB:Q15270",
  "term_id": "GO:0000978",
  "term_label": "RNA polymerase II cis-regulatory region sequence-specific DNA binding",
  "gene_symbol": "NKX1-1"
}